negative regulation of circulating fibrinogen levels [GO:0061754] (biological process) References: PMID:20570858 Sources: GOC:BHF, GOC:BHF_miRNA, GOC:rph Relationships: is a type of regulation of circulating fibrinogen levels [GO:0044537] Definition: Any process that reduces the quantity of fibrinogen circulating in the bloodstream.